{
  "gene_name": "Protein arginine N-methyltransferase 9",
  "gene": "UniProtKB:Q6P2P2",
  "term_label": "regulation of DNA-templated transcription",
  "gene_symbol": "PRMT9",
  "term_id": "GO:0006355"
}